{
  "gene": "UniProtKB:Q8TCG2",
  "term_label": "trans-Golgi network",
  "term_id": "GO:0005802",
  "gene_symbol": "PI4K2B",
  "gene_name": "Phosphatidylinositol 4-kinase type 2-beta"
}